{
  "gene_name": "Proprotein convertase subtilisin_kexin type 6",
  "term_id": "GO:0016486",
  "gene": "UniProtKB:P29122",
  "term_label": "peptide hormone processing",
  "gene_symbol": "PCSK6"
}